{
  "gene": "UniProtKB:Q8IUX4",
  "gene_name": "DNA dC-dU-editing enzyme APOBEC-3F",
  "term_id": "GO:0051607",
  "term_label": "defense response to virus",
  "gene_symbol": "APOBEC3F"
}